{
  "gene_symbol": "AKAIN1",
  "term_label": "Unknown biological process",
  "gene_name": "A-kinase anchor protein inhibitor 1",
  "term_id": "UNKNOWN:0002",
  "gene": "UniProtKB:P0CW23"
}